{
  "term_id": "GO:0009953",
  "gene_name": "Bone morphogenetic protein 1",
  "term_label": "dorsal/ventral pattern formation",
  "gene_symbol": "BMP1",
  "gene": "UniProtKB:P13497"
}